{
  "gene": "UniProtKB:P18850",
  "term_label": "endoplasmic reticulum unfolded protein response",
  "gene_name": "Cyclic AMP-dependent transcription factor ATF-6 alpha",
  "term_id": "GO:0030968",
  "gene_symbol": "ATF6"
}